{
  "gene": "UniProtKB:Q96S99",
  "term_id": "GO:0005769",
  "gene_symbol": "PLEKHF1",
  "gene_name": "Pleckstrin homology domain-containing family F member 1",
  "term_label": "early endosome"
}